{
  "term_label": "extracellular matrix",
  "gene_name": "Collagen alpha-1(XXIII) chain",
  "gene": "UniProtKB:Q86Y22",
  "term_id": "GO:0031012",
  "gene_symbol": "COL23A1"
}